glandular epithelial cell maturation [GO:0002071] (BP) Definition: The developmental process, independent of morphogenetic (shape) change, that is required for a glandular epithelial cell to attain its fully functional state. A glandular epithelial cell is a columnar/cuboidal epithelial cell is a cell found in a two dimensional sheet with a free surface exposed to the lumen of a gland. Sources: GOC:dph Relationships: is_a columnar/cuboidal epithelial cell maturation [GO:0002069]; BFO_0000050 glandular epithelial cell development [GO:0002068]